{
  "gene": "UniProtKB:Q9UPR0",
  "term_id": "GO:0048015",
  "gene_symbol": "PLCL2",
  "term_label": "phosphatidylinositol-mediated signaling",
  "gene_name": "Inactive phospholipase C-like protein 2"
}